RNA folding chaperone [GO:0140691] (molecular function) Definition: Binding to an RNA or an RNA-containing complex to assist the folding process. References: PMID:31165735 Relationships: is a type of molecular_function [GO:0003674]; is part of RNA folding [GO:0034337]